{
  "gene": "UniProtKB:Q15678",
  "gene_symbol": "PTPN14",
  "term_label": "positive regulation of hippo signaling",
  "gene_name": "Tyrosine-protein phosphatase non-receptor type 14",
  "term_id": "GO:0035332"
}